{
  "term_id": "GO:0002943",
  "gene_name": "tRNA-dihydrouridine(20) synthase [NAD(P)+]-like",
  "term_label": "tRNA dihydrouridine synthesis",
  "gene_symbol": "DUS2",
  "gene": "UniProtKB:Q9NX74"
}